{
  "gene_symbol": "PLEKHG5",
  "term_label": "endothelial cell migration",
  "gene_name": "Pleckstrin homology domain-containing family G member 5",
  "term_id": "GO:0043542",
  "gene": "UniProtKB:O94827"
}